beta-aspartyl-peptidase activity [GO:0008798] (molecular function) Definition: Catalysis of the cleavage of a beta-linked aspartic residue from the N-terminus of a polypeptide. Sources: EC:3.4.19.5 Also known as: beta-aspartyl dipeptidase activity, beta-aspartyl peptidase activity Relationships: is a type of omega peptidase activity [GO:0008242]; is a type of threonine-type peptidase activity [GO:0070003]